{
  "term_label": "cAMP-dependent protein kinase complex",
  "gene": "UniProtKB:P22694",
  "gene_symbol": "PRKACB",
  "gene_name": "cAMP-dependent protein kinase catalytic subunit beta",
  "term_id": "GO:0005952"
}